selenocysteine catabolic process [GO:0016261] (biological process) Definition: The chemical reactions and pathways resulting in the breakdown of selenocysteine, an essential component of glutathione peroxidase and some other proteins. Also known as: selenocysteine breakdown, selenocysteine catabolism, selenocysteine degradation Relationships: is_a selenocysteine metabolic process [GO:0016259]; is a type of GO:1901606 Sources: GOC:go_curators, ISBN:0198506732